{
  "term_label": "actin filament organization",
  "term_id": "GO:0007015",
  "gene": "UniProtKB:Q9BR76",
  "gene_symbol": "CORO1B",
  "gene_name": "Coronin-1B"
}